regulation of synapse structural plasticity [GO:0051823] (biological process) References: PMID:11063967, PMID:14976517, PMID:9884123 Also known as: regulation of synaptic structural plasticity Subtypes: negative regulation of synapse structural plasticity [GO:0051826], positive regulation of synapse structural plasticity [GO:0051835] Relationships: is a type of regulation of synapse organization [GO:0050807] Definition: Any process that modulates the frequency, rate or extent of synapse structural plasticity. Synapse structural plasticity is a type of cytoskeletal remodeling; this remodeling is induced by stimuli that can lead to long term potentiation and it can be activity-dependent or -independent. Examples of cytoskeletal changes include the formation of new spines and increase in spine size; this can be accompanied by the insertion of greater numbers of glutamate (or other neurotransmitter) receptors into the post-synaptic membrane.